regulation of plasma membrane sterol distribution [GO:0097036] (BP) Definition: Any process that modulates the proportions or spatial arrangement of sterols in the plasma membrane. References: PMID:18441123, PMID:20823909 Sources: GOC:mah Relationships: is a type of plasma membrane organization [GO:0007009]; is a type of regulation of membrane lipid distribution [GO:0097035]